{
  "term_label": "Unknown cellular component",
  "gene_symbol": "ZNF274",
  "term_id": "UNKNOWN:0003",
  "gene": "UniProtKB:Q96GC6",
  "gene_name": "Neurotrophin receptor-interacting factor homolog"
}